{
  "term_id": "GO:0030280",
  "gene": "UniProtKB:A0A140TA62",
  "gene_symbol": "LOC100653049",
  "gene_name": "IF rod domain-containing protein",
  "term_label": "structural constituent of skin epidermis"
}